{
  "gene_name": "Protocadherin gamma-A3",
  "gene_symbol": "PCDHGA3",
  "term_label": "plasma membrane",
  "gene": "UniProtKB:Q9Y5H0",
  "term_id": "GO:0005886"
}